{
  "gene_name": "CST complex subunit CTC1",
  "gene_symbol": "CTC1",
  "term_label": "CST complex",
  "term_id": "GO:1990879",
  "gene": "UniProtKB:Q2NKJ3"
}